{
  "gene": "UniProtKB:Q86UL3",
  "gene_symbol": "GPAT4",
  "gene_name": "Glycerol-3-phosphate acyltransferase 4",
  "term_label": "Unknown cellular component",
  "term_id": "UNKNOWN:0003"
}